{
  "gene_name": "Interleukin-27 subunit beta",
  "gene_symbol": "EBI3",
  "gene": "UniProtKB:Q14213",
  "term_label": "Unknown cellular component",
  "term_id": "UNKNOWN:0003"
}